{
  "gene_symbol": "SYN2",
  "gene_name": "Synapsin-2",
  "term_id": "GO:0030672",
  "term_label": "synaptic vesicle membrane",
  "gene": "UniProtKB:Q92777"
}